{
  "gene_symbol": "FLG2",
  "term_label": "keratohyalin granule",
  "gene_name": "Filaggrin-2",
  "gene": "UniProtKB:Q5D862",
  "term_id": "GO:0036457"
}